{
  "gene": "UniProtKB:Q96PX6",
  "gene_name": "Coiled-coil domain-containing protein 85A",
  "term_id": "UNKNOWN:0002",
  "term_label": "Unknown biological process",
  "gene_symbol": "CCDC85A"
}